{
  "gene_name": "Neuronal-specific septin-3",
  "gene_symbol": "SEPTIN3",
  "gene": "UniProtKB:Q9UH03",
  "term_label": "microtubule cytoskeleton",
  "term_id": "GO:0015630"
}